{
  "gene": "UniProtKB:Q13426",
  "term_label": "double-strand break repair via nonhomologous end joining",
  "term_id": "GO:0006303",
  "gene_name": "DNA repair protein XRCC4",
  "gene_symbol": "XRCC4"
}